{
  "term_id": "GO:0031209",
  "term_label": "SCAR complex",
  "gene_name": "Nck-associated protein 1",
  "gene": "UniProtKB:Q9Y2A7",
  "gene_symbol": "NCKAP1"
}